{
  "term_id": "UNKNOWN:0002",
  "gene_name": "Adenylate kinase 7",
  "term_label": "Unknown biological process",
  "gene_symbol": "AK7",
  "gene": "UniProtKB:Q96M32"
}